{
  "term_label": "fatty acid elongation, saturated fatty acid",
  "term_id": "GO:0019367",
  "gene_name": "Elongation of very long chain fatty acids protein 6",
  "gene": "UniProtKB:Q9H5J4",
  "gene_symbol": "ELOVL6"
}